{
  "gene_symbol": "TLR5",
  "gene_name": "Toll-like receptor 5",
  "term_id": "GO:0038023",
  "gene": "UniProtKB:O60602",
  "term_label": "signaling receptor activity"
}